{
  "gene": "UniProtKB:Q14773",
  "gene_name": "Intercellular adhesion molecule 4",
  "term_label": "integrin binding",
  "gene_symbol": "ICAM4",
  "term_id": "GO:0005178"
}